{
  "gene_name": "Cell surface glycoprotein CD200 receptor 1",
  "term_label": "Unknown biological process",
  "term_id": "UNKNOWN:0002",
  "gene": "UniProtKB:Q8TD46",
  "gene_symbol": "CD200R1"
}